{
  "term_label": "positive regulation of synaptic transmission, glutamatergic",
  "gene": "UniProtKB:O60359",
  "gene_symbol": "CACNG3",
  "gene_name": "Voltage-dependent calcium channel gamma-3 subunit",
  "term_id": "GO:0051968"
}